{
  "gene_symbol": "IKZF1",
  "term_label": "Unknown cellular component",
  "gene": "UniProtKB:Q13422",
  "gene_name": "DNA-binding protein Ikaros",
  "term_id": "UNKNOWN:0003"
}